{
  "term_label": "ESCRT I complex",
  "term_id": "GO:0000813",
  "gene_name": "Ubiquitin-associated protein 1",
  "gene": "UniProtKB:Q9NZ09",
  "gene_symbol": "UBAP1"
}